{
  "term_label": "negative regulation of Notch signaling pathway",
  "gene_name": "Delta-like protein 3",
  "gene_symbol": "DLL3",
  "term_id": "GO:0045746",
  "gene": "UniProtKB:Q9NYJ7"
}